{
  "gene_symbol": "MT1B",
  "term_id": "GO:0071294",
  "gene": "UniProtKB:P07438",
  "gene_name": "Metallothionein-1B",
  "term_label": "cellular response to zinc ion"
}